fusome organization [GO:0045478] (biological process) Relationships: is a type of organelle organization [GO:0006996]; is a type of GO:0022412 Subtypes: ovarian fusome organization [GO:0030723], GO:0030724 Definition: A process that is carried out at the cellular level which results in the assembly, arrangement of constituent parts, or disassembly of the fusome, a large intracellular spectrin-rich structure found in insect germline cells and mammalian hematopoietic cells. Also known as: fusome organisation, fusome organization and biogenesis Sources: GOC:dph, GOC:go_curators, GOC:jl, GOC:mah